mesangial cell differentiation [GO:0072007] (biological process) Sources: GOC:mtg_kidney_jan10 Definition: The process in which relatively unspecialized cells acquire specialized structural and/or functional features that characterize the mesangial cells of the kidney as it progresses from its formation to the mature state. Relationships: is a type of GO:0061005; is a type of GO:1904238 Subtypes: mesonephric mesangial cell differentiation [GO:0061260], glomerular mesangial cell differentiation [GO:0072008], metanephric mesangial cell differentiation [GO:0072209]